{
  "gene": "UniProtKB:Q9BTL3",
  "gene_symbol": "RAMAC",
  "term_id": "GO:0006370",
  "term_label": "7-methylguanosine mRNA capping",
  "gene_name": "RNA guanine-N7 methyltransferase activating subunit"
}